{
  "gene_name": "Bromodomain testis-specific protein",
  "term_id": "GO:0000785",
  "gene": "UniProtKB:Q58F21",
  "gene_symbol": "BRDT",
  "term_label": "chromatin"
}